{
  "term_id": "GO:0007267",
  "term_label": "cell-cell signaling",
  "gene": "UniProtKB:A6NN92",
  "gene_symbol": "GJE1",
  "gene_name": "Putative gap junction epsilon-1 protein"
}